regulation of root development [GO:2000280] (biological process) Sources: GOC:obol Definition: Any process that modulates the frequency, rate or extent of root development. Relationships: is a type of GO:0050793; regulates root development [GO:0048364] Subtypes: GO:2000069